cyclin E2-CDK2 complex [GO:0097135] (cellular component) References: PMID:15935619 Sources: GOC:so Relationships: is a type of cyclin-dependent protein kinase holoenzyme complex [GO:0000307] Definition: A protein complex consisting of cyclin E2 and cyclin-dependent kinase 2 (CDK2). Cyclins are characterized by periodicity in protein abundance throughout the cell cycle. Cyclin-dependent kinases represent a family of serine/threonine protein kinases that become active upon binding to a cyclin regulatory partner.